{
  "gene_symbol": "PARP9",
  "gene_name": "Protein mono-ADP-ribosyltransferase PARP9",
  "term_label": "NAD+ poly-ADP-ribosyltransferase activity",
  "term_id": "GO:0003950",
  "gene": "UniProtKB:Q8IXQ6"
}